{
  "gene": "UniProtKB:A6NGU5",
  "gene_name": "Putative glutathione hydrolase 3 proenzyme",
  "term_label": "regulation of inflammatory response",
  "term_id": "GO:0050727",
  "gene_symbol": "GGT3P"
}